{
  "gene_name": "Transcription factor ATOH1",
  "term_id": "GO:0005634",
  "gene": "UniProtKB:Q92858",
  "gene_symbol": "ATOH1",
  "term_label": "nucleus"
}